{
  "gene_name": "Cholesterol 25-hydroxylase",
  "gene_symbol": "CH25H",
  "term_id": "GO:0005789",
  "term_label": "endoplasmic reticulum membrane",
  "gene": "UniProtKB:O95992"
}